{
  "term_label": "plasma membrane",
  "gene_name": "FYN-binding protein 1",
  "gene_symbol": "FYB1",
  "term_id": "GO:0005886",
  "gene": "UniProtKB:O15117"
}